FH1 domain binding [GO:0017058] (molecular function) Sources: GOC:go_curators Relationships: is a type of protein domain specific binding [GO:0019904] Definition: Binding to a FH1 domain of a protein, a proline-rich domain, usually located in front of a FH2 domain.